{
  "term_id": "UNKNOWN:0002",
  "gene_name": "Serine_threonine-protein phosphatase CPPED1",
  "gene": "UniProtKB:Q9BRF8",
  "term_label": "Unknown biological process",
  "gene_symbol": "CPPED1"
}